{
  "gene": "UniProtKB:P26678",
  "term_id": "GO:0016020",
  "gene_name": "Cardiac phospholamban",
  "gene_symbol": "PLN",
  "term_label": "membrane"
}